{
  "term_id": "GO:0005815",
  "gene_name": "Cyclin-O",
  "gene": "UniProtKB:P22674",
  "gene_symbol": "CCNO",
  "term_label": "microtubule organizing center"
}